{
  "gene_symbol": "DARS1",
  "term_id": "GO:0005829",
  "term_label": "cytosol",
  "gene": "UniProtKB:P14868",
  "gene_name": "Aspartate--tRNA ligase, cytoplasmic"
}